{
  "term_label": "G protein-coupled receptor signaling pathway",
  "gene_symbol": "PLCB3",
  "gene": "UniProtKB:Q01970",
  "term_id": "GO:0007186",
  "gene_name": "1-phosphatidylinositol 4,5-bisphosphate phosphodiesterase beta-3"
}